{
  "gene_name": "Carcinoembryonic antigen-related cell adhesion molecule 1",
  "term_label": "protein tyrosine kinase binding",
  "gene": "UniProtKB:P13688",
  "gene_symbol": "CEACAM1",
  "term_id": "GO:1990782"
}